{
  "term_id": "GO:0005634",
  "gene_symbol": "HIVEP1",
  "gene_name": "Zinc finger protein 40",
  "term_label": "nucleus",
  "gene": "UniProtKB:P15822"
}